{
  "term_id": "GO:0005737",
  "term_label": "cytoplasm",
  "gene_symbol": "S100A7A",
  "gene": "UniProtKB:Q86SG5",
  "gene_name": "Protein S100-A7A"
}